{
  "term_id": "GO:0030425",
  "gene_name": "Spatacsin",
  "term_label": "dendrite",
  "gene": "UniProtKB:Q96JI7",
  "gene_symbol": "SPG11"
}